chitin-based larval cuticle pattern formation [GO:0035293] (biological process) Sources: GOC:bf, GOC:mtg_sensu Relationships: is a type of cuticle pattern formation [GO:0035017]; is part of larval chitin-based cuticle development [GO:0008363] Definition: The process that gives rise to the patterns of cell differentiation in the chitin-based larval cuticle. An example of this is found in Drosophila melanogaster.